{
  "term_id": "GO:0000132",
  "term_label": "establishment of mitotic spindle orientation",
  "gene_name": "Nuclear distribution protein nudE homolog 1",
  "gene": "UniProtKB:Q9NXR1",
  "gene_symbol": "NDE1"
}